{
  "gene_name": "Syntaxin-11",
  "term_label": "presynaptic active zone membrane",
  "gene": "UniProtKB:O75558",
  "gene_symbol": "STX11",
  "term_id": "GO:0048787"
}